cell-cell signaling involved in cardiac conduction [GO:0086019] (biological process) Relationships: is a type of GO:0007267; is a type of cell communication involved in cardiac conduction [GO:0086065] Subtypes: SA node cell to atrial cardiac muscle cell signaling [GO:0086018], atrial cardiac muscle cell to AV node cell signaling [GO:0086026], AV node cell to bundle of His cell signaling [GO:0086027], bundle of His cell to Purkinje myocyte signaling [GO:0086028], Purkinje myocyte to ventricular cardiac muscle cell signaling [GO:0086029] Definition: Any process that mediates the transfer of information from one cell to another and contributes to the heart process that regulates cardiac muscle contraction; beginning with the generation of an action potential in the sinoatrial node and ending with regulation of contraction of the myocardium. Sources: GOC:BHF, GOC:mtg_cardiac_conduct_nov11 Also known as: cell-cell signalling involved in cardiac conduction